{
  "gene": "UniProtKB:Q00597",
  "gene_symbol": "FANCC",
  "gene_name": "Fanconi anemia group C protein",
  "term_id": "GO:0043240",
  "term_label": "Fanconi anaemia nuclear complex"
}